alpha9-beta1 integrin-vascular cell adhesion molecule-1 complex [GO:0071065] (cellular component) Also known as: ITGA9-ITGB1-VCAM1 complex References: PMID:10209034 Definition: A protein complex that consists of an alpha9-beta1 integrin complex bound to vascular cell adhesion molecule-1. Relationships: is a type of plasma membrane protein complex [GO:0098797]